heat shock-mediated polytene chromosome puffing [GO:0035080] (biological process) Definition: The decondensing (loosening) and swelling of the chromosomal sites of heat shock genes on polytene chromosomes in response to a heat shock stimulus. Relationships: is a type of GO:0034605; is a type of polytene chromosome puffing [GO:0035079] References: PMID:12543962 Sources: GOC:bf